{
  "term_label": "perinuclear endoplasmic reticulum",
  "gene_symbol": "OSBPL7",
  "term_id": "GO:0097038",
  "gene": "UniProtKB:Q9BZF2",
  "gene_name": "Oxysterol-binding protein-related protein 7"
}